type 2 cannabinoid receptor binding [GO:0031719] (MF) Also known as: type 2 cannabinoid receptor ligand Sources: GOC:mah, GOC:nln Definition: Binding to a type 2 cannabinoid receptor. Relationships: is a type of cannabinoid receptor binding [GO:0031717]